establishment of protein localization to organelle [GO:0072594] (biological process) Definition: The directed movement of a protein to a specific location on or in an organelle. Encompasses establishment of localization in the membrane or lumen of a membrane-bounded organelle. Also known as: establishment of protein localisation to organelle Relationships: is a type of establishment of protein localization [GO:0045184] Sources: GOC:mah Subtypes: protein import into nucleus [GO:0006606], endocytic hemoglobin import into cell [GO:0020028], protein transmembrane import into intracellular organelle [GO:0044743], ubiquitin-dependent endocytosis [GO:0070086], GO:0070199, establishment of protein localization to spindle pole body [GO:0071989], establishment of protein localization to chloroplast [GO:0072596], establishment of protein localization to endoplasmic reticulum [GO:0072599], establishment of protein localization to mitochondrion [GO:0072655], establishment of protein localization to peroxisome [GO:0072663], establishment of protein localization to vacuole [GO:0072666], neurotransmitter receptor transport, plasma membrane to endosome [GO:0099646], GO:0140450